{
  "gene_symbol": "CRYGN",
  "term_id": "GO:0002088",
  "gene_name": "Gamma-crystallin N",
  "term_label": "lens development in camera-type eye",
  "gene": "UniProtKB:Q8WXF5"
}